{
  "term_label": "dynein light intermediate chain binding",
  "gene_name": "RILP-like protein 2",
  "gene_symbol": "RILPL2",
  "term_id": "GO:0051959",
  "gene": "UniProtKB:Q969X0"
}